{
  "gene_name": "Bromodomain-containing protein 4",
  "gene": "UniProtKB:O60885",
  "gene_symbol": "BRD4",
  "term_id": "GO:0005634",
  "term_label": "nucleus"
}